{
  "term_id": "GO:0072534",
  "gene_symbol": "HAPLN3",
  "term_label": "perineuronal net",
  "gene_name": "Hyaluronan and proteoglycan link protein 3",
  "gene": "UniProtKB:Q96S86"
}